{
  "term_label": "cytoplasm",
  "gene_symbol": "RNF115",
  "gene_name": "E3 ubiquitin-protein ligase RNF115",
  "gene": "UniProtKB:Q9Y4L5",
  "term_id": "GO:0005737"
}